MLL1 complex [GO:0071339] (cellular component) Definition: A protein complex that can methylate lysine-4 of histone H3. MLL1/MLL is the catalytic methyltransferase subunit, and the complex also contains the core components ASH2L, HCFC1/HCF1 WDR5 and RBBP5. Relationships: is a type of MLL1/2 complex [GO:0044665] References: PMID:15960975 Sources: GOC:sp